{
  "gene": "UniProtKB:Q96QD9",
  "gene_name": "UAP56-interacting factor",
  "gene_symbol": "FYTTD1",
  "term_id": "GO:0006406",
  "term_label": "mRNA export from nucleus"
}